{
  "term_label": "tumor necrosis factor-mediated signaling pathway",
  "gene": "UniProtKB:Q9Y6Q6",
  "gene_symbol": "TNFRSF11A",
  "term_id": "GO:0033209",
  "gene_name": "Tumor necrosis factor receptor superfamily member 11A"
}